{
  "term_label": "Unknown molecular function",
  "gene_name": "LASP1 neighbor protein",
  "term_id": "UNKNOWN:0001",
  "gene": "UniProtKB:A0A1B0GWH6",
  "gene_symbol": "LASP1NB"
}